{
  "gene": "UniProtKB:Q6NY19",
  "term_label": "cytoplasm",
  "gene_symbol": "KANK3",
  "term_id": "GO:0005737",
  "gene_name": "KN motif and ankyrin repeat domain-containing protein 3"
}